6-methylsalicylic acid synthase activity [GO:0050641] (molecular function) Definition: Catalysis of the reaction: acetyl-CoA + 3 H+ + 3 malonyl-CoA + NADPH = 6-methylsalicylate + 3 CO2 + 4 CoA + H2O + NADP+. Relationships: is a type of GO:0016747 Sources: EC:2.3.1.165, RHEA:12240 Also known as: 6-MSAS activity, MSAS activity, acyl-CoA:malonyl-CoA C-acyltransferase (decarboxylating, oxoacyl-reducing, thioester-hydrolysing and cyclizing)